{
  "gene_name": "Forkhead box protein O3B",
  "gene_symbol": "FOXO3B",
  "term_id": "GO:0006357",
  "gene": "UniProtKB:A0A2Z4LIS9",
  "term_label": "regulation of transcription by RNA polymerase II"
}